anatomical structure formation involved in morphogenesis [GO:0048646] (BP) Also known as: formation of an anatomical structure involved in morphogenesis Note: Note that, for example, the formation of a pseudopod in an amoeba would not be considered formation involved in morphogenesis because it would not be thought of as the formation of an anatomical structure that was part of the shaping of the amoeba during its development. The formation of an axon from a neuron would be considered the formation of an anatomical structure involved in morphogenesis because it contributes to the creation of the form of the neuron in a developmental sense. Definition: The developmental process pertaining to the initial formation of an anatomical structure from unspecified parts. This process begins with the specific processes that contribute to the appearance of the discrete structure and ends when the structural rudiment is recognizable. An anatomical structure is any biological entity that occupies space and is distinguished from its surroundings. Anatomical structures can be macroscopic such as a carpel, or microscopic such as an acrosome. Sources: GOC:dph, GOC:jid, GOC:tb Relationships: is a type of GO:0032502; is part of GO:0009653 Subtypes: angiogenesis [GO:0001525], GO:0001704, somitogenesis [GO:0001756], blastocyst formation [GO:0001825], neural fold formation [GO:0001842], lymphangiogenesis [GO:0001946], germinal center formation [GO:0002467], heart valve formation [GO:0003188], GO:0003207, endocardial cushion formation [GO:0003272], heart rudiment formation [GO:0003315], optic vesicle formation [GO:0003403], optic cup formation involved in camera-type eye development [GO:0003408], syncytium formation [GO:0006949], germarium-derived egg chamber formation [GO:0007293], cellularization [GO:0007349], GO:0007370, cephalic furrow formation [GO:0007376], amnioserosa formation [GO:0007378], nodulation [GO:0009877], GO:0010376, aerenchyma formation [GO:0010618], retina layer formation [GO:0010842], GO:0010927, neural rod formation [GO:0014023], neural keel formation [GO:0014025], notochord formation [GO:0014028], GO:0014029, prechordal plate formation [GO:0021501], neural fold elevation formation [GO:0021502], GO:0021504, floor plate formation [GO:0021508], roof plate formation [GO:0021509], central nervous system formation [GO:0021556], hindbrain formation [GO:0021576], medulla oblongata formation [GO:0021580], pons formation [GO:0021584], cerebellum formation [GO:0021588], rhombomere formation [GO:0021594], cranial nerve formation [GO:0021603], GO:0021684, GO:0021688, cerebellar Purkinje cell layer formation [GO:0021694], cerebellar cortex formation [GO:0021697], GO:0021705, inferior olivary nucleus formation [GO:0021715], superior olivary nucleus formation [GO:0021720], GO:0021819, neural plate formation [GO:0021990], lamina terminalis formation [GO:0021996], platelet formation [GO:0030220], GO:0030435, eggshell formation [GO:0030703], GO:0032475, arthrospore formation [GO:0034298], reproductive blastospore formation [GO:0034299], tube formation [GO:0035148], tracheal pit formation in open tracheal system [GO:0035202], selective angioblast sprouting [GO:0035474], dorsal motor nucleus of vagus nerve formation [GO:0035764], adrenal cortex formation [GO:0035802], tendon formation [GO:0035992], dorsal appendage formation [GO:0046843], chorion micropyle formation [GO:0046844], floral whorl formation [GO:0048458], flower formation [GO:0048460], animal organ formation [GO:0048645], anther wall tapetum formation [GO:0048656], adenohypophysis formation [GO:0048847], neurohypophysis formation [GO:0048849], hypophysis formation [GO:0048851], formation of anatomical boundary [GO:0048859], Spemann organizer formation [GO:0060061], limb bud formation [GO:0060174], GO:0060214, trabecula formation [GO:0060343], lung lobe formation [GO:0060464], GO:0060592, mammary gland bud formation [GO:0060615], GO:0060659, submandibular salivary gland formation [GO:0060661], labyrinthine layer formation [GO:0060714], ectodermal placode formation [GO:0060788], GO:0060900, taste bud formation [GO:0061195], GO:0061198, GO:0061554, cleistothecium formation [GO:0062248], GO:0071730, kidney rudiment formation [GO:0072003], renal vesicle formation [GO:0072033], GO:0072129, GO:0072187, blood microparticle formation [GO:0072564], GO:0075015, primitive streak formation [GO:0090009], leaflet formation [GO:0090014], anterior neural plate formation [GO:0090017], GO:0090018, amelogenesis [GO:0097186], dentinogenesis [GO:0097187], angiogenic sprout fusion [GO:0120077], morula formation [GO:0140001], apical ectodermal ridge formation [GO:1905139], tracheoesophageal septum formation [GO:1905327], plant organ formation [GO:1905393]